positive regulation of locomotion [GO:0040017] (biological process) Sources: GOC:go_curators Relationships: is a type of regulation of locomotion [GO:0040012]; is a type of positive regulation of biological process [GO:0048518]; positively regulates locomotion [GO:0040011] Definition: Any process that activates or increases the frequency, rate or extent of locomotion of a cell or organism. Also known as: up regulation of locomotion, up-regulation of locomotion, upregulation of locomotion, activation of locomotion, stimulation of locomotion Subtypes: positive regulation of chemotaxis [GO:0050921], GO:0090326, positive regulation of forward locomotion [GO:1905850], positive regulation of backward locomotion [GO:1905852], positive regulation of cell motility [GO:2000147]